{
  "term_label": "Cul3-RING ubiquitin ligase complex",
  "gene": "UniProtKB:Q9UJP4",
  "term_id": "GO:0031463",
  "gene_name": "Kelch-like protein 21",
  "gene_symbol": "KLHL21"
}